{
  "gene_symbol": "PKIB",
  "gene": "UniProtKB:Q9C010",
  "term_label": "cytoplasm",
  "gene_name": "cAMP-dependent protein kinase inhibitor beta",
  "term_id": "GO:0005737"
}